{
  "term_label": "protein kinase activator activity",
  "term_id": "GO:0030295",
  "gene_name": "MOB kinase activator 2",
  "gene_symbol": "MOB2",
  "gene": "UniProtKB:Q70IA6"
}